{
  "gene": "UniProtKB:Q96ND8",
  "term_label": "DNA-binding transcription factor activity, RNA polymerase II-specific",
  "gene_name": "Zinc finger protein 583",
  "term_id": "GO:0000981",
  "gene_symbol": "ZNF583"
}